extracellular matrix organization involved in endocardium development [GO:0061148] (biological process) Also known as: extracellular matrix organisation involved in endocardium development Sources: GOC:dph Definition: A process which results in the assembly, arrangement of constituent parts, or disassembly of an extracellular matrix of the endocardium. The endocardium is an anatomical structure comprised of an endothelium and an extracellular matrix that forms the innermost layer of tissue of the heart, and lines the heart chambers. Relationships: is a type of GO:0030198; is part of endocardium development [GO:0003157]